{
  "term_label": "recycling endosome membrane",
  "gene_name": "Leucine-zipper-like transcriptional regulator 1",
  "gene_symbol": "LZTR1",
  "gene": "UniProtKB:Q8N653",
  "term_id": "GO:0055038"
}